hyalurononglucosaminidase activity [GO:0004415] (molecular function) Definition: Catalysis of the random hydrolysis of (1->4) linkages between N-acetyl-beta-D-glucosamine and D-glucuronate residues in hyaluronate. Relationships: is a type of GO:0015929 Also known as: chondroitinase activity, hyaluronidase activity, hyaluronoglucosaminidase activity, chondroitinase I activity, hyaluronate 4-glycanohydrolase activity, hyaluronoglucosidase activity Sources: EC:3.2.1.35